{
  "gene": "UniProtKB:A1L168",
  "gene_symbol": "C20orf202",
  "term_id": "UNKNOWN:0003",
  "term_label": "Unknown cellular component",
  "gene_name": "Uncharacterized protein C20orf202"
}